visceral mesoderm-endoderm interaction involved in midgut development [GO:0007495] (biological process) Definition: The process of cell-cell signaling between visceral mesoderm cells and endoderm cells that is involved in the differentiation of cells in the midgut. Relationships: is a type of cell-cell signaling [GO:0007267]; is part of GO:0007494 Sources: GOC:dph, GOC:isa_complete Also known as: visceral mesoderm/endoderm interaction